renal water retention [GO:0003092] (biological process) Sources: GOC:mtg_cardio Also known as: negative regulation of renal water excretion Relationships: is a type of negative regulation of urine volume [GO:0035811] Definition: The process in which renal water excretion is decreased.